imaginal disc growth factor receptor binding [GO:0008084] (molecular function) Sources: GOC:mah Relationships: is a type of GO:0070851 Also known as: imaginal disc growth factor Definition: Binding to an imaginal disc growth factor receptor.